{
  "term_id": "UNKNOWN:0002",
  "gene_name": "Ubiquitin carboxyl-terminal hydrolase 45",
  "gene": "UniProtKB:Q70EL2",
  "term_label": "Unknown biological process",
  "gene_symbol": "USP45"
}